positive regulation of epithelial cell proliferation involved in lung morphogenesis [GO:0060501] (biological process) Subtypes: positive regulation of epithelial cell proliferation involved in lung bud dilation [GO:0060504] Definition: Any process that increases the rate or frequency of epithelial cell proliferation that results in the lung attaining its shape. Relationships: is a type of positive regulation of epithelial cell proliferation [GO:0050679]; is a type of GO:2000794; positively regulates epithelial cell proliferation involved in lung morphogenesis [GO:0060502] Sources: GOC:dph